protein localization to interphase microtubule organizing center [GO:1905509] (biological process) Definition: A process in which a protein is transported to, or maintained in, a location within an interphase microtubule organizing center. References: PMID:19001497 Sources: GOC:TermGenie, GO_REF:0000087 Also known as: protein localisation in interphase microtubule organizing center, protein localisation to interphase microtubule organizing center, protein localization in interphase microtubule organizing center Relationships: is a type of GO:1905508